negative regulation of bipolar cell growth [GO:0051517] (biological process) Definition: Any process that stops, prevents, or reduces the frequency, rate or extent of bipolar cell growth, polarized growth from both ends of a cell. Also known as: down regulation of bipolar cell growth, down-regulation of bipolar cell growth, downregulation of bipolar cell growth, inhibition of bipolar cell growth Subtypes: GO:0051520 Sources: GOC:ai Relationships: is a type of negative regulation of unidimensional cell growth [GO:0051511]; is a type of GO:0051516; negatively regulates bipolar cell growth [GO:0042815]